{
  "term_label": "chemorepellent activity",
  "gene": "UniProtKB:Q14563",
  "term_id": "GO:0045499",
  "gene_name": "Semaphorin-3A",
  "gene_symbol": "SEMA3A"
}